proteasome core complex assembly [GO:0080129] (biological process) Relationships: is a type of proteasome assembly [GO:0043248] References: PMID:12401807, PMID:17971041 Definition: The aggregation, arrangement and bonding together of a mature, active 20S proteasome core particle complex that does not contain any regulatory particles. Also known as: 20S proteasome assembly